cytoplasmic DNA replication factor C complex [GO:0043598] (cellular component) Relationships: is a type of DNA replication factor C complex [GO:0005663]; is part of GO:0043600 Also known as: cytoplasmic RFC, cytoplasmic clamp loader References: PMID:14646196, PMID:16172520 Sources: GOC:mtg_sensu Definition: A cytoplasmic complex of two polypeptides that loads the DNA polymerase processivity factor proliferating cell nuclear antigen (PCNA) onto DNA, thereby permitting processive DNA synthesis catalyzed by DNA polymerase. Examples of this component are found in prokaryotic species.